{
  "gene": "UniProtKB:Q6P1N0",
  "term_label": "RNA polymerase II cis-regulatory region sequence-specific DNA binding",
  "gene_name": "Coiled-coil and C2 domain-containing protein 1A",
  "term_id": "GO:0000978",
  "gene_symbol": "CC2D1A"
}